organic acid transport [GO:0015849] (biological process) Definition: The directed movement of organic acids, any acidic compound containing carbon in covalent linkage, into, out of or within a cell, or between cells, by means of some agent such as a transporter or pore. Subtypes: GO:0042918, carboxylic acid transport [GO:0046942] Relationships: is a type of transport [GO:0006810] Sources: ISBN:0198506732 Regulation: regulated by regulation of organic acid transport [GO:0032890]; negatively regulated by GO:0032891; positively regulated by positive regulation of organic acid transport [GO:0032892]